{
  "term_id": "GO:0005730",
  "gene_symbol": "MAK16",
  "gene": "UniProtKB:Q9BXY0",
  "gene_name": "Protein MAK16 homolog",
  "term_label": "nucleolus"
}